{
  "gene_symbol": "CTAG1A",
  "term_id": "UNKNOWN:0001",
  "gene": "UniProtKB:P78358",
  "gene_name": "Cancer_testis antigen 1",
  "term_label": "Unknown molecular function"
}